{
  "term_id": "UNKNOWN:0003",
  "gene_symbol": "A0A5F9ZGZ6",
  "term_label": "Unknown cellular component",
  "gene": "UniProtKB:A0A5F9ZGZ6",
  "gene_name": "Rho guanine nucleotide exchange factor 5_35 N-terminal domain-containing protein"
}